{
  "gene": "UniProtKB:P84022",
  "term_label": "I-SMAD binding",
  "gene_symbol": "SMAD3",
  "term_id": "GO:0070411",
  "gene_name": "Mothers against decapentaplegic homolog 3"
}